{
  "gene": "UniProtKB:Q9H7F0",
  "term_id": "GO:1902047",
  "gene_symbol": "ATP13A3",
  "gene_name": "Polyamine-transporting ATPase 13A3",
  "term_label": "polyamine transmembrane transport"
}